{
  "gene_symbol": "S100A8",
  "gene_name": "Protein S100-A8",
  "term_label": "leukocyte migration involved in inflammatory response",
  "term_id": "GO:0002523",
  "gene": "UniProtKB:P05109"
}